{
  "term_label": "cytosol",
  "gene": "UniProtKB:O60343",
  "gene_name": "TBC1 domain family member 4",
  "term_id": "GO:0005829",
  "gene_symbol": "TBC1D4"
}